{
  "gene_symbol": "CMBL",
  "term_label": "Unknown cellular component",
  "term_id": "UNKNOWN:0003",
  "gene": "UniProtKB:Q96DG6",
  "gene_name": "Carboxymethylenebutenolidase homolog"
}